{
  "gene_symbol": "METTL17",
  "gene_name": "Methyltransferase-like protein 17, mitochondrial",
  "term_label": "Unknown molecular function",
  "term_id": "UNKNOWN:0001",
  "gene": "UniProtKB:Q9H7H0"
}